fucoidanase activity [GO:0033909] (MF) References: PMID:11910806, PMID:6417453 Definition: Catalysis of the endohydrolysis of 1,2-alpha-L-fucoside linkages in fucoidan without release of sulfate. Relationships: is a type of hydrolase activity, hydrolyzing O-glycosyl compounds [GO:0004553] Also known as: poly(1,2-alpha-L-fucoside-4-sulfate) glycanohydrolase activity